{
  "gene_symbol": "DPYD",
  "gene_name": "Dihydropyrimidine dehydrogenase [NADP(+)]",
  "term_label": "dihydropyrimidine dehydrogenase (NADP+) activity",
  "term_id": "GO:0017113",
  "gene": "UniProtKB:Q12882"
}